{
  "gene_symbol": "TRIM74",
  "gene": "UniProtKB:Q86UV6",
  "term_id": "GO:0005737",
  "term_label": "cytoplasm",
  "gene_name": "Tripartite motif-containing protein 74"
}